{
  "term_id": "UNKNOWN:0001",
  "gene": "UniProtKB:P24043",
  "gene_symbol": "LAMA2",
  "gene_name": "Laminin subunit alpha-2",
  "term_label": "Unknown molecular function"
}